{
  "gene_symbol": "ACAT2",
  "gene_name": "Acetyl-CoA acetyltransferase, cytosolic",
  "term_id": "UNKNOWN:0002",
  "gene": "UniProtKB:Q9BWD1",
  "term_label": "Unknown biological process"
}